homeostasis of number of meristem cells [GO:0007639] (biological process) Relationships: is_a GO:0010075; is a type of homeostasis of number of cells within a tissue [GO:0048873] Definition: Any biological process involved in the maintenance of the steady-state number of cells within a population of cells in the meristem. Sources: GOC:isa_complete